{
  "gene_name": "Uncharacterized protein",
  "gene": "UniProtKB:A0A2R8YD15",
  "gene_symbol": "A0A2R8YD15",
  "term_id": "UNKNOWN:0002",
  "term_label": "Unknown biological process"
}